{
  "gene": "UniProtKB:Q13606",
  "gene_name": "Olfactory receptor 5I1",
  "gene_symbol": "OR5I1",
  "term_id": "GO:0005549",
  "term_label": "odorant binding"
}